{
  "gene_name": "Tektin-4",
  "term_id": "UNKNOWN:0001",
  "term_label": "Unknown molecular function",
  "gene_symbol": "TEKT4",
  "gene": "UniProtKB:Q8WW24"
}